mannosyl-oligosaccharide 1,6-alpha-mannosidase activity [GO:0052767] (molecular function) Definition: Catalysis of the hydrolysis of the alpha-(1->6) bonds of alpha-D-mannose residues in mannosyl-oligosaccharide. References: PMID:1849817, PMID:2338081 Sources: GOC:mengo_curators Also known as: 1,6-alpha-mannosidase activity, alpha-1,6-mannosidase activity, 1,6-alpha-mannosyl-oligosaccharide alpha-D-mannohydrolase activity, alpha-1,6-mannosyl-oligosaccharide alpha-D-mannohydrolase activity Relationships: is a type of GO:0015924